{
  "gene_symbol": "INVS",
  "term_label": "Unknown molecular function",
  "gene": "UniProtKB:Q9Y283",
  "term_id": "UNKNOWN:0001",
  "gene_name": "Inversin"
}